{
  "term_label": "Unknown molecular function",
  "gene_name": "Sperm protamine P1",
  "term_id": "UNKNOWN:0001",
  "gene_symbol": "PRM1",
  "gene": "UniProtKB:P04553"
}